{
  "term_label": "plasma membrane",
  "gene": "UniProtKB:Q9HC97",
  "term_id": "GO:0005886",
  "gene_symbol": "GPR35",
  "gene_name": "G-protein coupled receptor 35"
}